{
  "gene_symbol": "ZFP64",
  "gene_name": "Zinc finger protein 64",
  "term_label": "nucleus",
  "gene": "UniProtKB:Q9NTW7",
  "term_id": "GO:0005634"
}